{
  "term_id": "GO:0001227",
  "gene_name": "Homeobox protein TGIF2LX",
  "gene": "UniProtKB:Q8IUE1",
  "term_label": "DNA-binding transcription repressor activity, RNA polymerase II-specific",
  "gene_symbol": "TGIF2LX"
}